oxidoreductase activity, acting on CH or CH2 groups, oxygen as acceptor [GO:0016727] (molecular function) Definition: Catalysis of an oxidation-reduction (redox) reaction in which a CH2 group acts as a hydrogen or electron donor and reduces an oxygen molecule. Sources: GOC:ai Relationships: is a type of GO:0016725 Subtypes: xanthine oxidase activity [GO:0004855], 6-hydroxynicotinate dehydrogenase activity [GO:0043732], juglone 3-hydroxylase activity [GO:0050012], pteridine oxidase activity [GO:0050227], hypoxanthine oxidase activity [GO:0070675]